{
  "gene_symbol": "NRAS",
  "gene": "UniProtKB:P01111",
  "gene_name": "GTPase NRas",
  "term_label": "Ras protein signal transduction",
  "term_id": "GO:0007265"
}